{
  "gene_name": "TBC1 domain family member 2B",
  "gene": "UniProtKB:Q9UPU7",
  "term_id": "GO:0005737",
  "term_label": "cytoplasm",
  "gene_symbol": "TBC1D2B"
}